{
  "term_id": "GO:0005886",
  "gene": "UniProtKB:Q05193",
  "gene_symbol": "DNM1",
  "term_label": "plasma membrane",
  "gene_name": "Dynamin-1"
}